{
  "term_label": "N-acyltransferase activity",
  "gene_name": "Phospholipase A and acyltransferase 5",
  "gene": "UniProtKB:Q96KN8",
  "gene_symbol": "PLAAT5",
  "term_id": "GO:0016410"
}